{
  "term_label": "nuclear receptor-mediated steroid hormone signaling pathway",
  "gene_name": "Glucocorticoid receptor",
  "term_id": "GO:0030518",
  "gene_symbol": "NR3C1",
  "gene": "UniProtKB:P04150"
}